{
  "gene_symbol": "BAAT",
  "gene": "UniProtKB:Q14032",
  "term_id": "GO:0005777",
  "gene_name": "Bile acid-CoA:amino acid N-acyltransferase",
  "term_label": "peroxisome"
}